vacuolar protein processing [GO:0006624] (biological process) Also known as: vacuolar protein maturation, vacuolar proteolysis Definition: Protein processing that takes place in the vacuole. Most protein processing in the vacuole represents proteolytic cleavage of precursors to form active enzymes. Sources: GOC:mah Relationships: is a type of protein processing [GO:0016485]; occurs in vacuole [GO:0005773]